dorsal closure, amnioserosa morphology change [GO:0046664] (biological process) Definition: The changes that occur during dorsal closure of the shape and structure of the amnioserosa, an epithelium that occupies the dorsal side of the embryo. References: PMID:12147138 Relationships: is a type of embryonic morphogenesis [GO:0048598]; is a type of tissue morphogenesis [GO:0048729]; is part of dorsal closure [GO:0007391]